steroid binding [GO:0005496] (molecular function) Definition: Binding to a steroid, any of a large group of substances that have in common a ring system based on 1,2-cyclopentanoperhydrophenanthrene. Sources: GOC:jl, ISBN:0198506732 Relationships: is a type of GO:0008289 Subtypes: vitamin D binding [GO:0005499], sterol binding [GO:0032934], brassinosteroid binding [GO:0090411], lithocholic acid binding [GO:1902121], GO:1902122, 21-deoxycortisol binding [GO:1903877], 11beta-hydroxyprogesterone binding [GO:1903879], GO:1903880, estradiol binding [GO:1903924], GO:1990239